antigen processing and presentation of exogenous peptide antigen via MHC class II [GO:0019886] (biological process) Definition: The process in which an antigen-presenting cell expresses a peptide antigen of exogenous origin on its cell surface in association with an MHC class II protein complex. The peptide antigen is typically, but not always, processed from a whole protein. References: PMID:15771591 Sources: GOC:add, ISBN:0781735149 Relationships: is a type of antigen processing and presentation of exogenous peptide antigen [GO:0002478]; is a type of GO:0002495 Also known as: antigen presentation, exogenous antigen via MHC class II, antigen presentation, exogenous peptide antigen, antigen processing, exogenous antigen via major histocompatibility complex class II, exogenous peptide antigen processing and presentation via MHC class II